{
  "gene": "UniProtKB:Q96RB7",
  "term_label": "Unknown molecular function",
  "gene_name": "Olfactory receptor 5M11",
  "gene_symbol": "OR5M11",
  "term_id": "UNKNOWN:0001"
}